amino-acid racemase activity [GO:0047661] (molecular function) Also known as: L-amino acid racemase activity Relationships: is a type of racemase and epimerase activity, acting on amino acids and derivatives [GO:0016855] Definition: Catalysis of the reaction: an L-amino acid = a D-amino acid. Sources: EC:5.1.1.10, MetaCyc:AMINO-ACID-RACEMASE-RXN Subtypes: alanine racemase activity [GO:0008784], diaminopimelate epimerase activity [GO:0008837], glutamate racemase activity [GO:0008881], methionine racemase activity [GO:0018111], proline racemase activity [GO:0018112], lysine racemase activity [GO:0018113], threonine racemase activity [GO:0018114], serine racemase activity [GO:0030378], phenylalanine racemase (ATP-hydrolyzing) activity [GO:0047462], 4-hydroxyproline epimerase activity [GO:0047580], GO:0047679, aspartate racemase activity [GO:0047689], ornithine racemase activity [GO:0050157]